{
  "term_id": "GO:0007512",
  "gene_name": "Myosin-7",
  "gene": "UniProtKB:P12883",
  "gene_symbol": "MYH7",
  "term_label": "adult heart development"
}